11-hydroxythromboxane B2 dehydrogenase activity [GO:0036133] (molecular function) Definition: Catalysis of the reaction: thromboxane B2 + NAD+ = 11-dehydro-thromboxane B2 + NADH + H+. References: PMID:3461463, PMID:3823488, PMID:8200461 Sources: GOC:mw, KEGG_REACTION:R05060 Also known as: NAD dependent 11-hydroxythromboxane B2 dehydrogenase activity Note: Note that the KEGG_REACTION:R05060 reaction does not stipulate the acceptor group, and is therefore slightly more general than the activity described by GO:0036133. Relationships: is_a oxidoreductase activity, acting on the CH-CH group of donors, NAD or NADP as acceptor [GO:0016628]